negative regulation of gluconate transmembrane transport [GO:0035431] (BP) Definition: Any process that stops, prevents, or reduces the frequency, rate or extent of the directed movement of gluconate across a membrane by means of some agent such as a transporter or pore. Sources: GOC:vw Relationships: is a type of GO:0032891; is a type of negative regulation of transmembrane transport [GO:0034763]; is a type of regulation of gluconate transmembrane transport [GO:0035430]; negatively regulates gluconate transmembrane transport [GO:0035429] Also known as: down regulation of gluconate transport, down-regulation of gluconate transport, downregulation of gluconate transport, negative regulation of gluconate membrane transport, inhibition of gluconate transport, negative regulation of gluconate transport